{
  "gene_name": "Serine_threonine-protein kinase PAK 5",
  "term_label": "regulation of MAPK cascade",
  "gene": "UniProtKB:Q9P286",
  "gene_symbol": "PAK5",
  "term_id": "GO:0043408"
}